{
  "gene_symbol": "MEIS1",
  "gene_name": "Homeobox protein Meis1",
  "term_id": "GO:0001525",
  "term_label": "angiogenesis",
  "gene": "UniProtKB:O00470"
}